{
  "term_id": "GO:0019814",
  "term_label": "immunoglobulin complex",
  "gene": "UniProtKB:P01701",
  "gene_symbol": "IGLV1-51",
  "gene_name": "Immunoglobulin lambda variable 1-51"
}